{
  "gene_name": "HAUS augmin-like complex subunit 8",
  "term_label": "cytoplasm",
  "gene_symbol": "HAUS8",
  "gene": "UniProtKB:Q9BT25",
  "term_id": "GO:0005737"
}